{
  "gene_name": "Neutrophil cytosol factor 4",
  "gene_symbol": "NCF4",
  "term_id": "GO:0005737",
  "term_label": "cytoplasm",
  "gene": "UniProtKB:Q15080"
}